regulation of mesoderm formation [GO:1905902] (biological process) Definition: Any process that modulates the frequency, rate or extent of mesoderm formation. Subtypes: negative regulation of mesoderm formation [GO:1905903], GO:1905904 References: PMID:23939491 Sources: GOC:BHF, GOC:BHF_miRNA, GOC:TermGenie, GOC:rph, GO_REF:0000058 Relationships: is a type of regulation of developmental process [GO:0050793]; regulates mesoderm formation [GO:0001707]